{
  "term_label": "DNA damage tolerance",
  "gene_name": "Ubiquitin-conjugating enzyme E2 variant 2",
  "gene_symbol": "UBE2V2",
  "gene": "UniProtKB:Q15819",
  "term_id": "GO:0006301"
}